{
  "term_label": "Unknown cellular component",
  "term_id": "UNKNOWN:0003",
  "gene": "UniProtKB:Q96EI5",
  "gene_name": "Transcription elongation factor A protein-like 4",
  "gene_symbol": "TCEAL4"
}